heat acclimation [GO:0010286] (biological process) Subtypes: cellular heat acclimation [GO:0070370] Also known as: thermotolerance Definition: Any process that increases heat tolerance of an organism in response to high temperatures. Relationships: is a type of response to heat [GO:0009408] Sources: GOC:tair_curators